{
  "gene_name": "Tetraspanin-7",
  "gene_symbol": "TSPAN7",
  "term_id": "UNKNOWN:0001",
  "term_label": "Unknown molecular function",
  "gene": "UniProtKB:P41732"
}